{
  "term_label": "serine-type endopeptidase activity",
  "gene": "UniProtKB:Q5K4E3",
  "gene_symbol": "PRSS36",
  "term_id": "GO:0004252",
  "gene_name": "Polyserase-2"
}